{
  "term_label": "actin binding",
  "gene": "UniProtKB:P78559",
  "term_id": "GO:0003779",
  "gene_symbol": "MAP1A",
  "gene_name": "Microtubule-associated protein 1A"
}